{
  "gene_symbol": "WIPI1",
  "gene_name": "WD repeat domain phosphoinositide-interacting protein 1",
  "gene": "UniProtKB:Q5MNZ9",
  "term_label": "autophagy of mitochondrion",
  "term_id": "GO:0000422"
}